heme catabolic process [GO:0042167] (biological process) Subtypes: GO:0046157, heme a catabolic process [GO:0046161], heme C catabolic process [GO:0046163], heme O catabolic process [GO:0048035], heme B catabolic process [GO:1900548] Also known as: haem catabolic process, haem catabolism, heme breakdown, heme catabolism, heme degradation Relationships: is a type of porphyrin-containing compound catabolic process [GO:0006787]; is a type of heme metabolic process [GO:0042168]; is_a GO:0046149 Sources: GOC:jl Definition: The chemical reactions and pathways resulting in the breakdown of heme, any compound of iron complexed in a porphyrin (tetrapyrrole) ring.